analia development [GO:0007487] (biological process) Sources: GOC:ai, GOC:mtg_sensu Relationships: is a type of anatomical structure development [GO:0048856]; is part of genital disc development [GO:0035215] Subtypes: male analia development [GO:0045496], female analia development [GO:0045497] Definition: The process whose specific outcome is the progression of the analia over time, from its formation to the mature structure. The analia is the posterior-most vertral appendage that develops from the genital disc. An example of this process is analia development in Drosophila melanogaster.